{
  "term_label": "voltage-gated sodium channel complex",
  "gene_name": "Sodium channel protein type 9 subunit alpha",
  "gene_symbol": "SCN9A",
  "gene": "UniProtKB:Q15858",
  "term_id": "GO:0001518"
}